positive regulation of symbiont haustorium neck formation for entry into host [GO:0075199] (biological process) Note: Note that this term should not be used to annotate gene products of the host. It should only be used to annotate those gene products from the symbiont involved in this process. Relationships: is a type of GO:0051094; is a type of modulation of symbiont haustorium neck formation for entry into host [GO:0075198]; is a type of positive regulation by symbiont of entry into host [GO:0075294]; positively regulates GO:0075197 Sources: GOC:pamgo_curators Definition: Any process that activates, maintains or increases the frequency, rate or extent of symbiont haustorium neck formation for entry into host. The host is defined as the larger of the organisms involved in a symbiotic interaction.